{
  "gene_name": "CCR4-NOT transcription complex subunit 6-like",
  "gene_symbol": "CNOT6L",
  "gene": "UniProtKB:Q96LI5",
  "term_label": "3'-5'-RNA exonuclease activity",
  "term_id": "GO:0000175"
}